alginic acid catabolic process [GO:0042122] (biological process) Relationships: is a type of polysaccharide catabolic process [GO:0000272]; is a type of carboxylic acid catabolic process [GO:0046395] Sources: ISBN:0198506732 Also known as: alginate catabolic process, alginate catabolism, alginic acid breakdown, alginic acid catabolism, alginic acid degradation Definition: The chemical reactions and pathways resulting in the breakdown of alginic acid, a hydrophilic polysaccharide occurring in, for example, the cell walls of brown algae (brown seaweeds).